{
  "term_id": "GO:0035556",
  "gene": "UniProtKB:Q16659",
  "gene_symbol": "MAPK6",
  "term_label": "intracellular signal transduction",
  "gene_name": "Mitogen-activated protein kinase 6"
}